{
  "term_label": "keratinization",
  "gene_name": "Keratin, type II cuticular Hb1",
  "gene": "UniProtKB:Q14533",
  "gene_symbol": "KRT81",
  "term_id": "GO:0031424"
}